{
  "term_label": "Unknown biological process",
  "gene_symbol": "TTPAL",
  "gene": "UniProtKB:Q9BTX7",
  "term_id": "UNKNOWN:0002",
  "gene_name": "Alpha-tocopherol transfer protein-like"
}